{
  "gene_name": "Beta-1,4-mannosyl-glycoprotein 4-beta-N-acetylglucosaminyltransferase",
  "term_id": "GO:0016757",
  "gene": "UniProtKB:Q09327",
  "term_label": "glycosyltransferase activity",
  "gene_symbol": "MGAT3"
}